{
  "gene": "UniProtKB:A0A286YFG1",
  "term_id": "UNKNOWN:0002",
  "term_label": "Unknown biological process",
  "gene_name": "Small cysteine and glycine repeat-containing protein 8",
  "gene_symbol": "SCYGR8"
}